{
  "gene_name": "Sodium_glucose cotransporter 2",
  "term_label": "D-glucose:sodium symporter activity",
  "gene_symbol": "SLC5A2",
  "term_id": "GO:0005412",
  "gene": "UniProtKB:P31639"
}